{
  "gene_symbol": "TMCO5B",
  "term_id": "UNKNOWN:0001",
  "gene": "UniProtKB:A8MYB1",
  "term_label": "Unknown molecular function",
  "gene_name": "Transmembrane and coiled-coil domain-containing protein 5B"
}